{
  "term_id": "GO:0005634",
  "gene": "UniProtKB:P45984",
  "gene_symbol": "MAPK9",
  "gene_name": "Mitogen-activated protein kinase 9",
  "term_label": "nucleus"
}